{
  "term_id": "GO:0016064",
  "gene_name": "Immunoglobulin heavy variable 2-5",
  "term_label": "immunoglobulin mediated immune response",
  "gene_symbol": "IGHV2-5",
  "gene": "UniProtKB:P01817"
}